response to nerve growth factor [GO:1990089] (biological process) Subtypes: cellular response to nerve growth factor stimulus [GO:1990090] Relationships: is a type of response to growth factor [GO:0070848] References: PMID:22399805 Also known as: response to nerve growth factor stimulus Definition: A process that results in a change in state or activity of a cell or an organism (in terms of movement, secretion, enzyme production, gene expression, etc.) as a result of a nerve growth factor stimulus.